{
  "gene_symbol": "KLRC2",
  "gene_name": "NKG2-C type II integral membrane protein",
  "term_label": "activating MHC class Ib receptor activity",
  "term_id": "GO:0062081",
  "gene": "UniProtKB:P26717"
}